{
  "gene_name": "T cell receptor alpha joining 47 (Fragment)",
  "gene": "UniProtKB:A0A075B6Y5",
  "term_label": "Unknown cellular component",
  "gene_symbol": "TRAJ47",
  "term_id": "UNKNOWN:0003"
}